{
  "gene_symbol": "ARC",
  "term_id": "GO:0170047",
  "gene_name": "Activity-regulated cytoskeleton-associated protein",
  "gene": "UniProtKB:Q7LC44",
  "term_label": "virus-like capsid"
}